{
  "gene_symbol": "ITGB8",
  "gene_name": "Integrin beta-8",
  "term_id": "GO:0016477",
  "gene": "UniProtKB:P26012",
  "term_label": "cell migration"
}